{
  "term_label": "regulation of transcription by RNA polymerase II",
  "gene_symbol": "PROP1",
  "gene": "UniProtKB:O75360",
  "term_id": "GO:0006357",
  "gene_name": "Homeobox protein prophet of Pit-1"
}